{
  "gene_name": "Solute carrier family 22 member 3",
  "term_id": "UNKNOWN:0003",
  "term_label": "Unknown cellular component",
  "gene_symbol": "SLC22A3",
  "gene": "UniProtKB:O75751"
}